regulation of cilium movement involved in cell motility [GO:0060295] (biological process) Definition: Any process that modulates the rate frequency or extent of cilium movement involved in ciliary motility. Sources: GOC:BHF, GOC:dph, GOC:tb Relationships: is a type of regulation of cilium movement [GO:0003352]; is a type of regulation of cilium-dependent cell motility [GO:1902019]; regulates cilium movement involved in cell motility [GO:0060294] Subtypes: regulation of cilium beat frequency involved in ciliary motility [GO:0060296], regulation of flagellated sperm motility [GO:1901317]